{
  "term_label": "neuron projection",
  "term_id": "GO:0043005",
  "gene_name": "Microtubule-associated protein 2",
  "gene": "UniProtKB:P11137",
  "gene_symbol": "MAP2"
}